{
  "term_label": "ubiquitin-dependent protein catabolic process",
  "gene_name": "Ubiquitin-conjugating enzyme E2 H",
  "gene": "UniProtKB:P62256",
  "term_id": "GO:0006511",
  "gene_symbol": "UBE2H"
}